sodium-independent prostaglandin transport [GO:0071720] (biological process) Relationships: is_a prostaglandin transport [GO:0015732]; is a type of sodium-independent icosanoid transport [GO:0071718] Sources: GOC:krc Definition: The directed, sodium-independent, movement of prostaglandins into, out of or within a cell, or between cells, by means of some agent such as a transporter or pore.